{
  "term_id": "GO:0032190",
  "term_label": "acrosin binding",
  "gene": "UniProtKB:P60852",
  "gene_name": "Zona pellucida sperm-binding protein 1",
  "gene_symbol": "ZP1"
}